{
  "gene_name": "Hepatic and glial cell adhesion molecule",
  "gene_symbol": "HEPACAM",
  "term_label": "cell-cell junction",
  "gene": "UniProtKB:Q14CZ8",
  "term_id": "GO:0005911"
}